monoacylglycerol catabolic process [GO:0052651] (BP) Definition: The chemical reactions and pathways resulting in the breakdown of monoacylglycerol, any ester of glycerol in which any one of its hydroxyl groups has been acylated with a fatty acid, the other being non-esterified. References: PMID:25290914 Also known as: monoacylglycerol breakdown, monoacylglycerol catabolism, monoacylglycerol degradation Relationships: is_a monoacylglycerol metabolic process [GO:0046462]; is a type of acylglycerol catabolic process [GO:0046464]